{
  "gene": "UniProtKB:Q9BRH9",
  "term_id": "GO:0006357",
  "gene_name": "Zinc finger protein 251",
  "gene_symbol": "ZNF251",
  "term_label": "regulation of transcription by RNA polymerase II"
}